{
  "term_label": "Unknown biological process",
  "term_id": "UNKNOWN:0002",
  "gene_name": "Survival of motor neuron-related-splicing factor 30",
  "gene_symbol": "SMNDC1",
  "gene": "UniProtKB:O75940"
}